{
  "gene": "UniProtKB:Q96RP7",
  "gene_symbol": "GAL3ST4",
  "gene_name": "Galactose-3-O-sulfotransferase 4",
  "term_label": "Unknown cellular component",
  "term_id": "UNKNOWN:0003"
}